{
  "term_label": "protein-macromolecule adaptor activity",
  "gene_name": "Hematopoietic SH2 domain-containing protein",
  "gene": "UniProtKB:Q96JZ2",
  "term_id": "GO:0030674",
  "gene_symbol": "HSH2D"
}